{
  "term_id": "GO:0006457",
  "term_label": "protein folding",
  "gene_name": "Peptidyl-prolyl cis-trans isomerase E",
  "gene": "UniProtKB:Q9UNP9",
  "gene_symbol": "PPIE"
}